phosphatidate cytidylyltransferase activity [GO:0004605] (molecular function) Sources: EC:2.7.7.41 Definition: Catalysis of the reaction: CTP + phosphatidate = diphosphate + CDP-diacylglycerol. Also known as: CDP-diacylglycerol synthase activity, CDP-diglyceride diphosphorylase activity, CDP-diglyceride pyrophosphorylase activity, CDP-diglyceride synthase activity, CDP diglyceride pyrophosphorylase activity, CDP-DG, CDP-diacylglyceride synthetase activity, CDP-diglyceride synthetase activity, CTP-diacylglycerol synthetase activity, CTP:1,2-diacylglycerophosphate-cytidyl transferase activity, CTP:phosphatidate cytidylyltransferase activity, DAG synthetase activity, cytidine diphosphoglyceride pyrophosphorylase activity, phosphatidate cytidyltransferase activity, phosphatidic acid cytidylyltransferase activity Relationships: is a type of cytidylyltransferase activity [GO:0070567]